{
  "gene_symbol": "GNB2",
  "term_label": "cytoplasm",
  "gene": "UniProtKB:P62879",
  "term_id": "GO:0005737",
  "gene_name": "Guanine nucleotide-binding protein G(I)_G(S)_G(T) subunit beta-2"
}